positive regulation of rRNA processing [GO:2000234] (biological process) Sources: GOC:mah Relationships: is a type of GO:0051254; is a type of GO:2000232; positively regulates rRNA processing [GO:0006364] Also known as: positive regulation of 35S primary transcript processing Definition: Any process that activates or increases the frequency, rate or extent of rRNA processing.